enoyl-[acyl-carrier-protein] reductase (NADH) activity [GO:0004318] (molecular function) Definition: Catalysis of the reaction: a 2,3-saturated acyl-[ACP] + NAD+ = a (2E)-enoyl-[ACP] + H+ + NADH. Sources: RHEA:10240 Also known as: NADH-enoyl acyl carrier protein reductase activity, NADH-specific enoyl-ACP reductase activity, acyl-acyl-carrier-protein:NAD+ oxidoreductase, enoyl-ACP reductase (NADH) activity, enoyl-[acyl-carrier protein] reductase (NADH) activity, enoyl-acyl-carrier-protein reductase (NADH) Relationships: is a type of GO:0016631